tRNA 3'-end processing [GO:0042780] (biological process) Sources: GOC:go_curators Subtypes: tRNA 3'-terminal CCA addition [GO:0001680], mitochondrial tRNA 3'-end processing [GO:1990180] Relationships: is a type of GO:0008033; is a type of GO:0031123 Definition: The process in which the 3' end of a pre-tRNA molecule is converted to that of a mature tRNA. Also known as: tRNA 3' processing